bile-salt sulfotransferase activity [GO:0047704] (molecular function) Relationships: is a type of sulfotransferase activity [GO:0008146] Sources: EC:2.8.2.14, MetaCyc:BILE-SALT-SULFOTRANSFERASE-RXN Definition: Catalysis of the reaction: 3'-phosphoadenosine 5'-phosphosulfate + taurolithocholate = adenosine 3',5'-bisphosphate + taurolithocholate sulfate. Also known as: bile-salt sulphotransferase activity, BAST I activity, bile acid sulfotransferase I activity, glycolithocholate sulfotransferase activity, 3'-phosphoadenylyl-sulfate:glycolithocholate sulfotransferase activity, bile acid:3'-phosphoadenosine-5'-phosphosulfate sulfotransferase activity, bile salt:3'phosphoadenosine-5'-phosphosulfate:sulfotransferase activity